{
  "gene_symbol": "MSH6",
  "gene": "UniProtKB:P52701",
  "term_id": "GO:0032301",
  "term_label": "MutSalpha complex",
  "gene_name": "DNA mismatch repair protein Msh6"
}